{
  "term_id": "GO:0000977",
  "term_label": "RNA polymerase II transcription regulatory region sequence-specific DNA binding",
  "gene_symbol": "ZNF248",
  "gene": "UniProtKB:Q8NDW4",
  "gene_name": "Zinc finger protein 248"
}